maintenance of protein localization in organelle [GO:0072595] (biological process) Definition: Any process in which a protein is maintained in a specific location a specific location on or in an organelle, and is prevented from moving elsewhere. Encompasses establishment of localization in the membrane or lumen of a membrane-bounded organelle. Sources: GOC:mah Subtypes: maintenance of protein localization in endoplasmic reticulum [GO:0035437], maintenance of protein location in nucleus [GO:0051457], maintenance of protein location to spindle pole body [GO:0071990], GO:0072597, maintenance of protein location in mitochondrion [GO:0072656], maintenance of protein location in peroxisome [GO:0072664], GO:0072667 Relationships: is a type of GO:0032507; is part of protein localization to organelle [GO:0033365]; occurs in organelle [GO:0043226] Also known as: maintenance of protein localisation to organelle, maintenance of protein localization to organelle